{
  "gene_name": "Cis-aconitate decarboxylase",
  "term_id": "GO:0050728",
  "term_label": "negative regulation of inflammatory response",
  "gene_symbol": "ACOD1",
  "gene": "UniProtKB:A6NK06"
}